{
  "term_label": "neuropeptide hormone activity",
  "gene_symbol": "ASIP",
  "gene": "UniProtKB:P42127",
  "term_id": "GO:0005184",
  "gene_name": "Agouti-signaling protein"
}